penicillin metabolic process [GO:0042316] (biological process) Definition: The chemical reactions and pathways involving any antibiotic that contains the condensed beta-lactamthiazolidine ring system. Penicillins are produced naturally during the growth of various microfungi of the genera Penicillium and Aspergillus. Sources: GOC:jl, ISBN:0198506732 Also known as: penicillin metabolism Relationships: is a type of GO:0006790; is a type of secondary metabolic process [GO:0019748]; is a type of monocarboxylic acid metabolic process [GO:0032787]; is a type of lactam metabolic process [GO:0072338] Subtypes: penicillin catabolic process [GO:0042317], GO:0042318, benzylpenicillin metabolic process [GO:1901086] Regulation: positively regulated by positive regulation of penicillin metabolic process [GO:0033246]